chemosensory behavior [GO:0007635] (biological process) Subtypes: chemosensory jump behavior [GO:0007636], proboscis extension reflex [GO:0007637], olfactory behavior [GO:0042048], behavioral response to chemical pain [GO:0061366] Sources: GOC:go_curators Also known as: behavioral response to chemical stimulus, behavioural response to chemical stimulus, chemosensory behaviour Relationships: is a type of behavior [GO:0007610]; is part of response to chemical [GO:0042221] Definition: Behavior that is dependent upon the sensation of chemicals.